{
  "gene": "UniProtKB:Q9UHD9",
  "gene_name": "Ubiquilin-2",
  "gene_symbol": "UBQLN2",
  "term_label": "autophagosome assembly",
  "term_id": "GO:0000045"
}